{
  "term_id": "GO:0005737",
  "gene": "UniProtKB:P04733",
  "gene_symbol": "MT1F",
  "gene_name": "Metallothionein-1F",
  "term_label": "cytoplasm"
}